{
  "gene": "UniProtKB:Q13470",
  "term_id": "UNKNOWN:0002",
  "gene_name": "Non-receptor tyrosine-protein kinase TNK1",
  "term_label": "Unknown biological process",
  "gene_symbol": "TNK1"
}